{
  "term_label": "tRNA cytidine N4-acetyltransferase activity",
  "gene_symbol": "NAT10",
  "gene_name": "RNA cytidine acetyltransferase",
  "gene": "UniProtKB:Q9H0A0",
  "term_id": "GO:0051392"
}